{
  "gene_symbol": "EHD4",
  "gene": "UniProtKB:Q9H223",
  "term_id": "GO:0072659",
  "gene_name": "EH domain-containing protein 4",
  "term_label": "protein localization to plasma membrane"
}